{
  "gene_symbol": "DLG2",
  "term_id": "GO:0098609",
  "term_label": "cell-cell adhesion",
  "gene": "UniProtKB:Q15700",
  "gene_name": "Disks large homolog 2"
}